retrograde vesicle-mediated transport, Golgi to endoplasmic reticulum [GO:0006890] (biological process) Subtypes: vesicle targeting, cis-Golgi to rough endoplasmic reticulum [GO:0048206] Also known as: cis-Golgi to rough ER transport, cis-Golgi to rough ER vesicle-mediated transport, cis-Golgi to rough endoplasmic reticulum transport, cis-Golgi to rough endoplasmic reticulum vesicle-mediated transport, retrograde (Golgi to ER) transport, retrograde transport, Golgi to ER, retrograde transport, Golgi to endoplasmic reticulum, retrograde vesicle-mediated transport, Golgi to ER Regulation: RO_0002211 by regulation of retrograde vesicle-mediated transport, Golgi to ER [GO:2000156] References: PMID:16510524 Sources: ISBN:0716731363 Definition: The directed movement of substances from the Golgi back to the endoplasmic reticulum, mediated by vesicles bearing specific protein coats such as COPI or COG. Relationships: is a type of Golgi vesicle transport [GO:0048193]